dUMP kinase activity [GO:0120136] (molecular function) Also known as: ATP:dUMP phosphotransferase activity, dUMP-kinase activity, deoxyuridine monophosphate kinase activity References: PMID:3010881 Sources: RHEA:30655 Definition: Catalysis of the reaction: ATP + dUMP = ADP + dUDP. Relationships: is_a deoxynucleoside phosphate kinase activity, ATP as phosphate donor [GO:0047507]